{
  "gene": "UniProtKB:Q9UKP4",
  "term_label": "proteolysis",
  "gene_name": "A disintegrin and metalloproteinase with thrombospondin motifs 7",
  "gene_symbol": "ADAMTS7",
  "term_id": "GO:0006508"
}